{
  "term_id": "GO:0005096",
  "gene_symbol": "RGS16",
  "gene_name": "Regulator of G-protein signaling 16",
  "gene": "UniProtKB:O15492",
  "term_label": "GTPase activator activity"
}